post-spliceosomal complex [GO:0071020] (cellular component) Also known as: mammalian spliceosomal complex C2, yeast spliceosomal complex A2-3 Relationships: is a type of GO:0005681; BFO_0000051 U5 snRNP [GO:0005682] Sources: GOC:krc, GOC:mah, ISBN:0879695897, ISBN:0879697393 Subtypes: U2-type post-spliceosomal complex [GO:0071021], U12-type post-spliceosomal complex [GO:0071022] Definition: A spliceosomal complex that is formed following the second splicing event and contains the spliced product, the excised intron, and three snRNPs, including U5.